AGG codon-amino acid adaptor activity [GO:0033448] (MF) Sources: GOC:mah Note: Note that in the standard genetic code, AGG codes for arginine. Relationships: is a type of triplet codon-amino acid adaptor activity [GO:0030533] Definition: A triplet codon-amino acid adaptor activity that recognizes an AGG codon. Also known as: arginine tRNA